pyrimidine ribonucleoside triphosphate metabolic process [GO:0009208] (biological process) Definition: The chemical reactions and pathways involving pyrimidine ribonucleoside triphosphate, a compound consisting of a pyrimidine base linked to a ribose sugar esterified with triphosphate on the sugar. Also known as: pyrimidine ribonucleoside triphosphate metabolism Sources: GOC:go_curators, ISBN:0198506732 Subtypes: pyrimidine ribonucleoside triphosphate biosynthetic process [GO:0009209], pyrimidine ribonucleoside triphosphate catabolic process [GO:0009210], CTP metabolic process [GO:0046036], GO:0046046, GO:0046051 Relationships: is a type of pyrimidine nucleoside triphosphate metabolic process [GO:0009147]